{
  "term_label": "plasma membrane",
  "term_id": "GO:0005886",
  "gene": "UniProtKB:P20020",
  "gene_name": "Plasma membrane calcium-transporting ATPase 1",
  "gene_symbol": "ATP2B1"
}